{
  "term_label": "icosanoid biosynthetic process",
  "gene": "UniProtKB:Q5TCH4",
  "term_id": "GO:0046456",
  "gene_name": "Cytochrome P450 4A22",
  "gene_symbol": "CYP4A22"
}